{
  "gene": "UniProtKB:P28799",
  "gene_symbol": "GRN",
  "gene_name": "Progranulin",
  "term_label": "Unknown molecular function",
  "term_id": "UNKNOWN:0001"
}